{
  "term_id": "GO:0008397",
  "gene_name": "7-alpha-hydroxycholest-4-en-3-one 12-alpha-hydroxylase",
  "term_label": "sterol 12-alpha-hydroxylase activity",
  "gene_symbol": "CYP8B1",
  "gene": "UniProtKB:Q9UNU6"
}